{
  "gene_name": "tRNA (adenine(58)-N(1))-methyltransferase catalytic subunit TRMT61A",
  "gene_symbol": "TRMT61A",
  "term_label": "tRNA (m1A) methyltransferase complex",
  "gene": "UniProtKB:Q96FX7",
  "term_id": "GO:0031515"
}